replication fork arrest at rDNA repeats [GO:0031582] (biological process) Also known as: replication fork arrest at ribosomal DNA repeats, replication fork blocking at rDNA repeats Sources: GOC:mah, GOC:vw Definition: A process that impedes the progress of the DNA replication fork at natural replication fork pausing sites within the eukaryotic rDNA repeat spacer. Relationships: is a type of maintenance of rDNA [GO:0043007]; is a type of GO:0043111 Regulation: RO_0002211 by regulation of replication fork arrest at rDNA repeats [GO:1902681]